{
  "term_label": "axon guidance",
  "gene": "UniProtKB:Q9C0C4",
  "gene_name": "Semaphorin-4C",
  "gene_symbol": "SEMA4C",
  "term_id": "GO:0007411"
}